transmitter-gated monoatomic ion channel activity [GO:0022824] (molecular function) Sources: GOC:mtg_transport, ISBN:0815340729 Definition: Enables the transmembrane transfer of an ion by a channel that opens when a specific neurotransmitter has been bound by the channel complex or one of its constituent parts. Relationships: is a type of extracellular ligand-gated monoatomic ion channel activity [GO:0005230]; is a type of transmitter-gated channel activity [GO:0022835] Also known as: transmitter-gated ion channel activity, ionotropic neurotransmitter receptor activity Subtypes: glutamate-gated receptor activity [GO:0004970], serotonin-gated monoatomic cation channel activity [GO:0022850], GABA-gated chloride ion channel activity [GO:0022851], GO:0022852, GO:0160039, glycine-gated cation channel activity [GO:0160212], transmitter-gated monoatomic ion channel activity involved in regulation of postsynaptic membrane potential [GO:1904315]